{
  "term_label": "recycling endosome",
  "gene_symbol": "DENND6A",
  "gene": "UniProtKB:Q8IWF6",
  "gene_name": "Protein DENND6A",
  "term_id": "GO:0055037"
}